{
  "term_id": "GO:0000977",
  "gene_symbol": "ZNF487",
  "term_label": "RNA polymerase II transcription regulatory region sequence-specific DNA binding",
  "gene_name": "Putative zinc finger protein 487",
  "gene": "UniProtKB:B1APH4"
}